{
  "term_id": "UNKNOWN:0001",
  "term_label": "Unknown molecular function",
  "gene": "UniProtKB:Q9UPZ6",
  "gene_symbol": "THSD7A",
  "gene_name": "Thrombospondin type-1 domain-containing protein 7A"
}